intracellular protein transport [GO:0006886] (biological process) Sources: GOC:mah Definition: The directed movement of proteins in a cell, including the movement of proteins between specific compartments or structures within a cell, such as organelles of a eukaryotic cell. Also known as: copper-induced intracellular protein transport Regulation: regulated by GO:0033157; positively regulated by positive regulation of intracellular protein transport [GO:0090316]; negatively regulated by negative regulation of intracellular protein transport [GO:0090317] Relationships: is a type of protein transport [GO:0015031]; is a type of intracellular transport [GO:0046907]; BFO_0000050 GO:0008104 Subtypes: protein import into nucleus [GO:0006606], protein export from nucleus [GO:0006611], GO:0006623, GO:0007038, GO:0015869, protein exit from endoplasmic reticulum [GO:0032527], protein transport within lipid bilayer [GO:0032594], GO:0033369, GO:0033376, protein transport to vacuole involved in ubiquitin-dependent protein catabolic process via the multivesicular body sorting pathway [GO:0043328], GO:0045046, intracellular protein transmembrane transport [GO:0065002], misfolded protein transport [GO:0070843], polyubiquitinated protein transport [GO:0070844], protein transport along microtubule [GO:0098840], neurotransmitter receptor transport, postsynaptic endosome to lysosome [GO:0098943], microtubule polymerization based protein transport [GO:0099112], endosome to plasma membrane protein transport [GO:0099638]